A2A adenosine receptor binding [GO:0031687] (molecular function) Sources: GOC:mah, GOC:nln Also known as: A2A adenosine receptor ligand Relationships: is a type of adenosine receptor binding [GO:0031685] Definition: Binding to an A2A adenosine receptor.